{
  "gene_name": "Phosphorylase b kinase regulatory subunit beta",
  "term_label": "Unknown biological process",
  "gene_symbol": "PHKB",
  "term_id": "UNKNOWN:0002",
  "gene": "UniProtKB:Q93100"
}